response to humidity [GO:0009270] (biological process) Relationships: is a type of response to water [GO:0009415] Definition: Any process that results in a change in state or activity of a cell or an organism (in terms of movement, secretion, enzyme production, gene expression, etc.) as a result of a humidity stimulus, moisture in the atmosphere. Subtypes: cellular response to humidity [GO:0071463], GO:0090547 Sources: GOC:jl